{
  "gene_name": "Tigger transposable element-derived protein 6",
  "term_label": "DNA binding",
  "term_id": "GO:0003677",
  "gene_symbol": "TIGD6",
  "gene": "UniProtKB:Q17RP2"
}